mitochondrial inner membrane peptidase complex [GO:0042720] (cellular component) References: PMID:10821182, PMID:12191769 Relationships: is a type of inner mitochondrial membrane protein complex [GO:0098800]; is_a serine-type endopeptidase complex [GO:1905370] Also known as: mitochondrion inner membrane peptidase complex, IMP Definition: Protease complex of the mitochondrial inner membrane, consisting of at least two subunits, involved in processing of both nuclear- and mitochondrially-encoded proteins targeted to the intermembrane space.